T cell lineage commitment [GO:0002360] (biological process) Relationships: is a type of GO:0045165; is part of T cell differentiation [GO:0030217] Sources: GOC:add, ISBN:0781735149 Subtypes: alpha-beta T cell lineage commitment [GO:0002363], gamma-delta T cell lineage commitment [GO:0002365], CD4-positive or CD8-positive, alpha-beta T cell lineage commitment [GO:0043369] Also known as: T lymphocyte lineage commitment, T-cell lineage commitment, T-lymphocyte lineage commitment Definition: The process in which a lymphoid progenitor cell becomes committed to becoming any type of T cell.